{
  "gene_name": "Mitochondrial coenzyme A transporter SLC25A42",
  "term_label": "Unknown biological process",
  "term_id": "UNKNOWN:0002",
  "gene_symbol": "SLC25A42",
  "gene": "UniProtKB:Q86VD7"
}